{
  "term_label": "Unknown molecular function",
  "gene_symbol": "MRPL48",
  "gene": "UniProtKB:Q96GC5",
  "gene_name": "Large ribosomal subunit protein mL48",
  "term_id": "UNKNOWN:0001"
}